{
  "gene": "UniProtKB:Q96MA1",
  "gene_symbol": "DMRTB1",
  "gene_name": "Doublesex- and mab-3-related transcription factor B1",
  "term_id": "GO:0000978",
  "term_label": "RNA polymerase II cis-regulatory region sequence-specific DNA binding"
}